{
  "term_label": "cytoplasm",
  "gene_name": "15-hydroxyprostaglandin dehydrogenase [NAD(+)]",
  "gene_symbol": "HPGD",
  "term_id": "GO:0005737",
  "gene": "UniProtKB:P15428"
}